type IV secretion system complex [GO:0043684] (CC) Relationships: is_a GO:0032991 Sources: GOC:ml Also known as: T4SS complex, type IV protein secretion system complex Definition: A complex of proteins related to those involved in bacterial DNA conjugative transfer, that permits the transfer of DNA or proteins into the extracellular milieu or directly into host cells. In general the type IV complex forms a multisubunit cell-envelope-spanning structure composed of a secretion channel and often a pilus or other surface filament or protein(s).